{
  "gene": "UniProtKB:Q8NH89",
  "gene_name": "Putative olfactory receptor 5AK3",
  "term_id": "GO:0005549",
  "gene_symbol": "OR5AK3P",
  "term_label": "odorant binding"
}